diadenosine tetraphosphate biosynthetic process [GO:0015966] (biological process) Definition: The chemical reactions and pathways resulting in the formation of diadenosine tetraphosphate, a derivative of the nucleoside adenosine with four phosphate groups attached. Relationships: is a type of GO:0015960 Sources: GOC:ai Also known as: diadenosine tetraphosphate anabolism, diadenosine tetraphosphate biosynthesis, diadenosine tetraphosphate formation, diadenosine tetraphosphate synthesis